{
  "gene_name": "ALK and LTK ligand 2",
  "gene": "UniProtKB:Q6UX46",
  "term_id": "UNKNOWN:0003",
  "gene_symbol": "ALKAL2",
  "term_label": "Unknown cellular component"
}